{
  "gene_name": "Receptor-transporting protein 4",
  "term_id": "GO:0031849",
  "term_label": "olfactory receptor binding",
  "gene": "UniProtKB:Q96DX8",
  "gene_symbol": "RTP4"
}